detoxification of free heme [GO:0140725] (biological process) Also known as: free heme detoxification References: PMID:26741528, PMID:32983129 Definition: Any process that reduces or removes the toxicity of free heme. These include transport of heme away from sensitive areas and to compartments or complexes whose purpose is sequestration of heme. Relationships: is a type of GO:0098754